lipopolysaccharide transmembrane transporter activity [GO:0015221] (molecular function) Also known as: LPS transmembrane transporter activity Definition: Enables the transfer of lipopolysaccharides from one side of a membrane to the other. A lipopolysaccharide is any of a group of related, structurally complex components of the outer membrane of Gram-negative bacteria. Lipopolysaccharides consist three covalently linked regions, lipid A, core oligosaccharide, and an O side chain. Lipid A is responsible for the toxicity of the lipopolysaccharide. Relationships: is a type of macromolecule transmembrane transporter activity [GO:0022884]; is_a lipid transmembrane transporter activity [GO:0170055]; is_a GO:1901505; BFO_0000050 GO:0015920 Sources: GOC:ai, GOC:mtg_transport, ISBN:0815340729